autophagic cell death [GO:0048102] (biological process) Also known as: autophagic death, programmed cell death by autophagy, programmed cell death by macroautophagy, autosis, type II programmed cell death Regulation: regulated by regulation of autophagic cell death [GO:1904092]; negatively regulated by negative regulation of autophagic cell death [GO:1904093]; positively regulated by GO:1904094 Relationships: is a type of programmed cell death [GO:0012501]; has part GO:0016236 Note: The precise nature of autophagic cell death is still being debated, and the link between autophagy and cell death unclear. As autophagy is often induced under conditions of stress that could also lead to cell death, there has been a propagation of the idea that autophagy can act as a cell death mechanism; but others suggest that autophagy may simply be an attempt of dying cells to adapt to lethal stress rather than a mechanism to execute a cell death program. Further studies are required to resolve this controversy (see e.g. PMID:22082964, PMID:22052193, PMID:25236395). In the meantime, curators should carefully examine the experimental evidence presented in papers concerning autophagic cell death, and annotate accordingly. Recently, an instance of autophagic cell death, termed autosis, was discovered that relies on the plasma membrane Na+/K+-ATPase. Autosis was observed in vivo in the brain of rats subjected to an ischemic insult. It's still unclear if all cases of autophagic cell death require the Na+/K+-ATPase or not. Definition: A form of programmed cell death that is accompanied by the formation of autophagosomes. Autophagic cell death is characterized by lack of chromatin condensation and massive vacuolization of the cytoplasm, with little or no uptake by phagocytic cells. References: PMID:18846107, PMID:23347517 Sources: GOC:autophagy, GOC:mah, GOC:mtg_apoptosis